{
  "gene_name": "Zinc finger protein 770",
  "term_id": "GO:0006357",
  "gene": "UniProtKB:Q6IQ21",
  "term_label": "regulation of transcription by RNA polymerase II",
  "gene_symbol": "ZNF770"
}